{
  "gene_symbol": "EREG",
  "gene_name": "Proepiregulin",
  "gene": "UniProtKB:O14944",
  "term_id": "GO:0005154",
  "term_label": "epidermal growth factor receptor binding"
}